{
  "gene_symbol": "FOXL1",
  "gene": "UniProtKB:Q12952",
  "term_id": "GO:0006357",
  "gene_name": "Forkhead box protein L1",
  "term_label": "regulation of transcription by RNA polymerase II"
}